{
  "gene_name": "Homeobox protein DLX-2",
  "term_id": "GO:0048706",
  "term_label": "embryonic skeletal system development",
  "gene_symbol": "DLX2",
  "gene": "UniProtKB:Q07687"
}